{
  "gene_symbol": "RAB14",
  "term_label": "early endosome",
  "gene": "UniProtKB:P61106",
  "gene_name": "Ras-related protein Rab-14",
  "term_id": "GO:0005769"
}